{
  "gene": "UniProtKB:P00734",
  "gene_name": "Prothrombin",
  "gene_symbol": "F2",
  "term_label": "extracellular matrix",
  "term_id": "GO:0031012"
}